protein localization to chloroplast starch grain [GO:1904160] (biological process) Also known as: protein localisation in chloroplast starch grain, protein localisation to chloroplast starch grain, protein localization in chloroplast starch grain References: PMID:25710501 Sources: GOC:TermGenie, GO_REF:0000087 Definition: A process in which a protein is transported to, or maintained in, a location within a chloroplast starch grain. Relationships: is a type of protein localization to chloroplast [GO:0072598]